{
  "term_label": "Unknown molecular function",
  "gene_symbol": "TMEM260",
  "gene_name": "Transmembrane protein 260",
  "gene": "UniProtKB:Q9NX78",
  "term_id": "UNKNOWN:0001"
}